{
  "term_id": "GO:0031410",
  "gene_name": "Occludin_ELL domain-containing protein 1",
  "gene_symbol": "OCEL1",
  "term_label": "cytoplasmic vesicle",
  "gene": "UniProtKB:Q9H607"
}